endosomal pattern recognition receptor signaling pathway [GO:0002754] (biological process) Also known as: intracellular endosomal pattern recognition receptor signaling pathway, intracellular vesicle PAMP receptor signaling pathway, intracellular vesicle PRR signaling pathway, intracellular vesicle pathogen receptor signaling pathway, intracellular vesicle pattern recognition receptor signaling pathway, intracellular vesicle pattern recognition receptor signalling pathway Relationships: is_a cytoplasmic pattern recognition receptor signaling pathway [GO:0002753] References: PMID:15199967 Sources: GOC:add, GOC:ar, ISBN:0781735149 Definition: The series of molecular signals initiated by the binding of a ligand to an intracellular vesicle pattern recognition receptor (PRR). PRRs bind pathogen-associated molecular pattern (PAMPs), structures conserved among microbial species.